{
  "term_label": "guanyl-nucleotide exchange factor activity",
  "gene_symbol": "RASGRF1",
  "term_id": "GO:0005085",
  "gene_name": "Ras-specific guanine nucleotide-releasing factor 1",
  "gene": "UniProtKB:Q13972"
}